{
  "term_id": "GO:0005654",
  "gene_symbol": "DTX2",
  "gene_name": "Probable E3 ubiquitin-protein ligase DTX2",
  "term_label": "nucleoplasm",
  "gene": "UniProtKB:Q86UW9"
}